formic acid secretion [GO:0046721] (biological process) Definition: The controlled release of formic acid, HCOOH, by a cell or a tissue. Also known as: formate secretion Sources: GOC:ai Relationships: is a type of formate transport [GO:0015724]; is a type of acid secretion [GO:0046717]